{
  "gene": "UniProtKB:Q9Y5X0",
  "gene_name": "Sorting nexin-10",
  "term_id": "GO:0016050",
  "gene_symbol": "SNX10",
  "term_label": "vesicle organization"
}